{
  "gene_symbol": "ATP6V0C",
  "gene": "UniProtKB:P27449",
  "term_id": "UNKNOWN:0002",
  "gene_name": "V-type proton ATPase 16 kDa proteolipid subunit c",
  "term_label": "Unknown biological process"
}